{
  "gene": "UniProtKB:Q9H808",
  "gene_symbol": "TLE6",
  "term_id": "GO:0005634",
  "term_label": "nucleus",
  "gene_name": "Transducin-like enhancer protein 6"
}